long-chain fatty acid binding [GO:0036041] (molecular function) Note: While there is not universal consensus on the lengths of short-, medium-, long- and very-long-chain fatty acids, the GO uses the definitions in ChEBI (see CHEBI:26666, CHEBI:59554, CHEBI:15904 and CHEBI:27283). Definition: Binding to a long-chain fatty acid. A long-chain fatty acid has an aliphatic tail containing 13 to 22 carbons. Relationships: is a type of fatty acid binding [GO:0005504] Also known as: long chain fatty acid binding Subtypes: icosatetraenoic acid binding [GO:0050543], GO:0050646, GO:0050647, GO:0050648, oleic acid binding [GO:0070538], GO:0070539, stearic acid binding [GO:0070540], GO:1904769 References: PMID:12641450 Sources: GOC:pm